{
  "gene_symbol": "SNRPN",
  "term_label": "U5 snRNP",
  "term_id": "GO:0005682",
  "gene": "UniProtKB:P63162",
  "gene_name": "Small nuclear ribonucleoprotein-associated protein N"
}